regulation of opsonization [GO:1903027] (biological process) Relationships: is a type of regulation of immune effector process [GO:0002697]; is a type of regulation of cellular process [GO:0050794]; regulates opsonization [GO:0008228] References: PMID:22333221 Sources: GOC:BHF, GOC:TermGenie, GOC:rl, GO_REF:0000058 Definition: Any process that modulates the frequency, rate or extent of opsonization. Subtypes: positive regulation of opsonization [GO:1903028]